female germline stem cell symmetric division [GO:0062102] (biological process) References: PMID:30248087 Sources: GOC:ha Relationships: is a type of germline stem cell symmetric division [GO:0098729] Definition: Division of a female germline stem cell to produce two germline stem cells of the same type as the parent.